{
  "gene_name": "Peroxisomal succinyl-coenzyme A thioesterase",
  "term_label": "peroxisome",
  "gene_symbol": "ACOT4",
  "gene": "UniProtKB:Q8N9L9",
  "term_id": "GO:0005777"
}